{
  "term_label": "positive regulation of cytosolic calcium ion concentration",
  "gene_name": "C-X-C chemokine receptor type 5",
  "gene_symbol": "CXCR5",
  "gene": "UniProtKB:P32302",
  "term_id": "GO:0007204"
}